{
  "gene": "UniProtKB:Q13574",
  "term_label": "diacylglycerol metabolic process",
  "gene_symbol": "DGKZ",
  "gene_name": "Diacylglycerol kinase zeta",
  "term_id": "GO:0046339"
}